{
  "term_label": "wound healing",
  "gene_symbol": "DST",
  "gene": "UniProtKB:Q03001",
  "gene_name": "Dystonin",
  "term_id": "GO:0042060"
}